negative regulation of kinetochore assembly [GO:1905560] (biological process) Definition: Any process that stops, prevents or reduces the frequency, rate or extent of kinetochore assembly. Also known as: down regulation of kinetochore assembly, down regulation of kinetochore biogenesis, down-regulation of kinetochore assembly, downregulation of kinetochore assembly, down regulation of centromere and kinetochore complex maturation, down regulation of centromere/kinetochore complex maturation, down regulation of chromosome-kinetochore attachment, down-regulation of centromere and kinetochore complex maturation, down-regulation of centromere/kinetochore complex maturation, down-regulation of chromosome-kinetochore attachment, downregulation of centromere and kinetochore complex maturation, downregulation of centromere/kinetochore complex maturation, downregulation of chromosome-kinetochore attachment, inhibition of centromere and kinetochore complex maturation, inhibition of centromere/kinetochore complex maturation, inhibition of chromosome-kinetochore attachment, inhibition of kinetochore assembly, negative regulation of NMS complex assembly, negative regulation of centromere and kinetochore complex maturation, negative regulation of centromere/kinetochore complex maturation, negative regulation of chromosome-kinetochore attachment, down regulation of kinetochore formation, down-regulation of kinetochore formation, downregulation of kinetochore formation, inhibition of kinetochore formation, negative regulation of kinetochore formation Relationships: is a type of GO:0031333; is a type of regulation of kinetochore assembly [GO:0090234]; is a type of negative regulation of organelle assembly [GO:1902116]; is a type of negative regulation of chromosome organization [GO:2001251]; negatively regulates GO:0051382 References: PMID:18765790 Sources: GOC:TermGenie, GO_REF:0000058